{
  "gene_name": "Eukaryotic translation initiation factor 1b",
  "gene_symbol": "EIF1B",
  "gene": "UniProtKB:O60739",
  "term_label": "eukaryotic 43S preinitiation complex",
  "term_id": "GO:0016282"
}